arginine-tRNA ligase activity [GO:0004814] (molecular function) Sources: EC:6.1.1.19 Also known as: arginyl-tRNA synthetase activity, L-arginine:tRNAArg ligase (AMP-forming), arginine translase activity, arginine-tRNA synthetase activity, arginyl transfer ribonucleic acid synthetase activity, arginyl-transfer RNA synthetase activity, arginyl-transfer ribonucleate synthetase activity Relationships: is a type of aminoacyl-tRNA ligase activity [GO:0004812] Definition: Catalysis of the reaction: ATP + L-arginine + tRNA(Arg) = AMP + diphosphate + L-arginyl-tRNA(Arg).